{
  "gene_name": "Ras-related protein Rab-33B",
  "gene": "UniProtKB:Q9H082",
  "term_id": "GO:0005794",
  "gene_symbol": "RAB33B",
  "term_label": "Golgi apparatus"
}